{
  "term_label": "alpha-(1->3)-fucosyltransferase activity",
  "term_id": "GO:0046920",
  "gene_name": "Alpha-(1,3)-fucosyltransferase 11",
  "gene": "UniProtKB:Q495W5",
  "gene_symbol": "FUT11"
}